{
  "gene": "UniProtKB:P01286",
  "gene_name": "Somatoliberin",
  "term_id": "GO:0016608",
  "term_label": "growth hormone-releasing hormone activity",
  "gene_symbol": "GHRH"
}